{
  "gene_name": "Fibroblast growth factor 14",
  "term_id": "GO:0005634",
  "gene_symbol": "FGF14",
  "gene": "UniProtKB:Q92915",
  "term_label": "nucleus"
}